{
  "term_label": "glycine receptor clustering",
  "gene_symbol": "GPHN",
  "gene": "UniProtKB:Q9NQX3",
  "term_id": "GO:0072579",
  "gene_name": "Gephyrin"
}